{
  "gene": "UniProtKB:Q6PIZ9",
  "term_id": "UNKNOWN:0001",
  "gene_name": "T-cell receptor-associated transmembrane adapter 1",
  "gene_symbol": "TRAT1",
  "term_label": "Unknown molecular function"
}